{
  "term_id": "GO:0003777",
  "term_label": "microtubule motor activity",
  "gene_symbol": "KIF4B",
  "gene_name": "Chromosome-associated kinesin KIF4B",
  "gene": "UniProtKB:Q2VIQ3"
}